oviduct morphogenesis [GO:0035848] (biological process) Also known as: fallopian tube morphogenesis Definition: The process in which anatomical structures of the oviduct are generated and organized. An oviduct is a tube through which an ova passes from the ovary to the uterus, or from the ovary to the outside of the organism. References: PMID:22918811 Sources: GOC:yaf Relationships: is a type of animal organ morphogenesis [GO:0009887]; is a type of GO:0035239; is part of oviduct development [GO:0060066]